{
  "gene_symbol": "ARL14",
  "term_label": "plasma membrane",
  "term_id": "GO:0005886",
  "gene": "UniProtKB:Q8N4G2",
  "gene_name": "ADP-ribosylation factor-like protein 14"
}